positive regulation of uterine smooth muscle relaxation [GO:1900721] (biological process) Also known as: activation of smooth muscle relaxation of the uterus, positive regulation of smooth muscle relaxation of the uterus, up regulation of smooth muscle relaxation of the uterus, up regulation of uterine smooth muscle relaxation, up-regulation of smooth muscle relaxation of the uterus, up-regulation of uterine smooth muscle relaxation, upregulation of smooth muscle relaxation of the uterus, upregulation of uterine smooth muscle relaxation, activation of uterine smooth muscle relaxation Relationships: is a type of regulation of uterine smooth muscle relaxation [GO:1900719]; is a type of GO:1901082; positively regulates GO:0044558 Definition: Any process that activates or increases the frequency, rate or extent of uterine smooth muscle relaxation. Sources: GOC:TermGenie